{
  "gene_symbol": "PACSIN2",
  "gene": "UniProtKB:Q9UNF0",
  "term_id": "GO:0030100",
  "gene_name": "Protein kinase C and casein kinase substrate in neurons protein 2",
  "term_label": "regulation of endocytosis"
}